oxidoreductase activity, acting on the CH-NH2 group of donors, cytochrome as acceptor [GO:0016640] (molecular function) Definition: Catalysis of an oxidation-reduction (redox) reaction in which a CH-NH2 group acts as a hydrogen or electron donor and reduces a cytochrome molecule. Relationships: is a type of GO:0016638 Subtypes: glycine dehydrogenase (cytochrome) activity [GO:0047959] Sources: GOC:ai